cellular response to chromate [GO:0071247] (biological process) Definition: Any process that results in a change in state or activity of a cell (in terms of movement, secretion, enzyme production, gene expression, etc.) as a result of a chromate stimulus. Sources: GOC:mah Relationships: is a type of GO:0046687; is a type of cellular response to oxygen-containing compound [GO:1901701]